{
  "term_id": "GO:0006508",
  "gene_name": "Pepsin A-3",
  "gene": "UniProtKB:P0DJD8",
  "gene_symbol": "PGA3",
  "term_label": "proteolysis"
}